response to puromycin [GO:1905794] (biological process) Definition: Any process that results in a change in state or activity of a cell or an organism (in terms of movement, secretion, enzyme production, gene expression, etc.) as a result of a puromycin stimulus. References: PMID:25736288 Sources: GOC:TermGenie, GO_REF:0000071 Relationships: is a type of GO:0014074; is a type of response to oxygen-containing compound [GO:1901700] Also known as: response to 3'-deoxy-N,N-dimethyl-3'-(O-methyl-L-tyrosinamido)adenosine Subtypes: cellular response to puromycin [GO:1905795]